{
  "gene_name": "Olfactory receptor 5D18",
  "gene": "UniProtKB:Q8NGL1",
  "term_id": "UNKNOWN:0003",
  "gene_symbol": "OR5D18",
  "term_label": "Unknown cellular component"
}